{
  "term_label": "inflammatory response",
  "gene": "UniProtKB:P49137",
  "term_id": "GO:0006954",
  "gene_symbol": "MAPKAPK2",
  "gene_name": "MAP kinase-activated protein kinase 2"
}